response to biotin [GO:0070781] (BP) Also known as: response to Bios IIB, response to coenzyme R, response to vitamin B7, response to vitamin H Relationships: is a type of GO:0033273; is a type of GO:1901698; is a type of response to oxygen-containing compound [GO:1901700] Subtypes: cellular response to biotin [GO:0071296] Sources: GOC:sl Definition: Any process that results in a change in state or activity of a cell or an organism (in terms of movement, secretion, enzyme production, gene expression, etc.) as a result of a biotin stimulus.